{
  "gene_symbol": "ODF3L2",
  "gene_name": "Outer dense fiber protein 3-like protein 2",
  "term_label": "Unknown molecular function",
  "gene": "UniProtKB:Q3SX64",
  "term_id": "UNKNOWN:0001"
}